primitive streak formation [GO:0090009] (BP) Definition: The developmental process pertaining to the initial formation of the primitive streak from unspecified parts. The primitive streak is a ridge of cells running along the midline of the embryo where the mesoderm ingresses. It defines the anterior-posterior axis. Relationships: is a type of anatomical structure formation involved in morphogenesis [GO:0048646]; is part of gastrulation with mouth forming second [GO:0001702]; is part of anterior/posterior axis specification [GO:0009948] Sources: GOC:dph, GOC:sdb_2009, GOC:tb